{
  "term_id": "UNKNOWN:0001",
  "gene_symbol": "INSYN2B",
  "gene": "UniProtKB:A6NMK8",
  "term_label": "Unknown molecular function",
  "gene_name": "Protein INSYN2B"
}